{
  "term_label": "neuronal cell body",
  "gene_symbol": "PDYN",
  "term_id": "GO:0043025",
  "gene": "UniProtKB:P01213",
  "gene_name": "Proenkephalin-B"
}